{
  "term_id": "GO:0000785",
  "gene_symbol": "PIAS2",
  "gene_name": "E3 SUMO-protein ligase PIAS2",
  "gene": "UniProtKB:O75928",
  "term_label": "chromatin"
}